{
  "gene": "UniProtKB:Q53H96",
  "term_label": "pyrroline-5-carboxylate reductase activity",
  "term_id": "GO:0004735",
  "gene_name": "Pyrroline-5-carboxylate reductase 3",
  "gene_symbol": "PYCR3"
}